osteoblast proliferation [GO:0033687] (biological process) Regulation: regulated by regulation of osteoblast proliferation [GO:0033688]; negatively regulated by negative regulation of osteoblast proliferation [GO:0033689]; positively regulated by positive regulation of osteoblast proliferation [GO:0033690] Definition: The multiplication or reproduction of osteoblasts, resulting in the expansion of an osteoblast cell population. An osteoblast is a bone-forming cell which secretes an extracellular matrix. Hydroxyapatite crystals are then deposited into the matrix to form bone. Relationships: is a type of cell population proliferation [GO:0008283] Sources: GOC:mah